mitotic checkpoint complex assembly [GO:1905660] (biological process) Definition: The aggregation, arrangement and bonding together of a set of components to form a mitotic checkpoint complex. Relationships: is a type of protein-containing complex assembly [GO:0065003] Also known as: MCC assembly, MCC formation, mitotic checkpoint complex formation References: PMID:26882497 Sources: GOC:TermGenie, GO_REF:0000079